{
  "gene_symbol": "FRMD4B",
  "term_label": "Unknown molecular function",
  "term_id": "UNKNOWN:0001",
  "gene": "UniProtKB:Q9Y2L6",
  "gene_name": "FERM domain-containing protein 4B"
}